negative regulation of hexasaccharide transport [GO:1900298] (biological process) Relationships: is a type of negative regulation of transport [GO:0051051]; is a type of regulation of hexasaccharide transport [GO:1900297]; negatively regulates GO:2001102 Sources: GOC:TermGenie, GOC:mengo_curators Also known as: down regulation of hexasaccharide transport, down-regulation of hexasaccharide transport, downregulation of hexasaccharide transport, inhibition of hexasaccharide transport Definition: Any process that stops, prevents or reduces the frequency, rate or extent of hexasaccharide transport. Subtypes: negative regulation of maltohexaose transport [GO:1900313]